rhamnulose-1-phosphate aldolase activity [GO:0008994] (molecular function) Relationships: is a type of aldehyde-lyase activity [GO:0016832] Also known as: L-rhamnulose 1-phosphate aldolase activity, L-rhamnulose-1-phosphate S-lactaldehyde-lyase (glycerone-phosphate-forming), L-rhamnulose-1-phosphate lactaldehyde-lyase activity, L-rhamnulose-phosphate aldolase activity, rhamnulose phosphate aldolase activity Sources: EC:4.1.2.19 Definition: Catalysis of the reaction: L-rhamnulose 1-phosphate = glycerone phosphate + (S)-lactaldehyde.